phosphothreonine residue binding [GO:0050816] (MF) Relationships: is a type of GO:0045309 Also known as: phosphothreonine binding Sources: GOC:ai Definition: Binding to a phosphorylated threonine residue within a protein.